{
  "term_label": "transmembrane transporter binding",
  "term_id": "GO:0044325",
  "gene": "UniProtKB:Q6ZRF8",
  "gene_symbol": "RNF207",
  "gene_name": "RING finger protein 207"
}